{
  "term_id": "GO:0051011",
  "term_label": "microtubule minus-end binding",
  "gene_name": "HAUS augmin-like complex subunit 4",
  "gene": "UniProtKB:Q9H6D7",
  "gene_symbol": "HAUS4"
}